dihydrofolate biosynthetic process [GO:0006761] (biological process) Sources: GOC:ai Relationships: is a type of folic acid-containing compound biosynthetic process [GO:0009396]; is a type of dicarboxylic acid biosynthetic process [GO:0043650]; is a type of dihydrofolate metabolic process [GO:0046452] Definition: The chemical reactions and pathways resulting in the formation of dihydrofolate, the dihydroxylated derivative of folate. Also known as: 7,8-dihydrofolate biosynthesis, 7,8-dihydrofolate biosynthetic process, dihydrofolate anabolism, dihydrofolate biosynthesis, dihydrofolate formation, dihydrofolate synthesis